{
  "term_label": "rRNA processing",
  "term_id": "GO:0006364",
  "gene_symbol": "DDX54",
  "gene_name": "ATP-dependent RNA helicase DDX54",
  "gene": "UniProtKB:Q8TDD1"
}